nucleolar exosome (RNase complex) [GO:0101019] (cellular component) Relationships: is a type of nuclear exosome (RNase complex) [GO:0000176]; is part of nucleolus [GO:0005730] Definition: A ribonuclease complex that has 3-prime to 5-prime distributive hydrolytic exoribonuclease activity and in some taxa (e.g. yeast) endoribonuclease activity, producing 5-prime-phosphomonoesters. Participates in a multitude of cellular RNA processing and degradation events preventing nuclear export and/or translation of aberrant RNAs. Restricted to processing linear and circular single-stranded RNAs (ssRNA) only. RNAs with complex secondary structures may have to be unwound or pre-processed by co-factors prior to entering the complex, esp if the 3-prime end is structured. References: PMID:17174896, PMID:20531386, PMID:26726035